amyloid-beta formation [GO:0034205] (biological process) Regulation: regulated by GO:1902003; positively regulated by positive regulation of amyloid-beta formation [GO:1902004]; negatively regulated by GO:1902430 Relationships: is a type of GO:0042987; is a type of amyloid-beta metabolic process [GO:0050435] Note: Note that this term does not fall under the general GO definition for biosynthetic processes, which is 'The chemical reactions and pathways resulting in the formation of... ', because amyloid-beta can only be formed by the proteolysis of a larger molecule (see term definition). The word 'formation' is therefore used in place of biosynthesis. Also, note that this term refers to the production of the amyloid-beta polypeptide from the amyloid precursor protein (APP), and should be used to annotate e.g. secretases that cleave APP to form amyloid-beta. To annotate gene products involved in the formation of amyloid fibrils, please consider 'amyloid fibril formation' (GO:1990000). Also known as: beta-amyloid formation, beta-amyloid polypeptide formation from APP, beta-amyloid polypeptide formation from amyloid precursor protein Definition: The generation of amyloid-beta by cleavage of the amyloid precursor protein (APP). Sources: GOC:mah